{
  "gene": "UniProtKB:Q9BT09",
  "term_id": "UNKNOWN:0002",
  "gene_symbol": "CNPY3",
  "term_label": "Unknown biological process",
  "gene_name": "Protein canopy homolog 3"
}